{
  "term_label": "cell-cell junction assembly",
  "gene_symbol": "CDH22",
  "term_id": "GO:0007043",
  "gene": "UniProtKB:Q9UJ99",
  "gene_name": "Cadherin-22"
}